{
  "gene_symbol": "NPR3",
  "gene_name": "Atrial natriuretic peptide receptor 3",
  "term_label": "Unknown cellular component",
  "gene": "UniProtKB:P17342",
  "term_id": "UNKNOWN:0003"
}